hippocampus development [GO:0021766] (biological process) Definition: The progression of the hippocampus over time from its initial formation until its mature state. Also known as: hippocampal formation development Relationships: is a type of GO:0048856; is part of GO:0021543; is part of limbic system development [GO:0021761] Sources: GOC:cls, GOC:dgh, GOC:dph, GOC:jid, GO_REF:0000021